vinorine synthase activity [GO:0050636] (molecular function) Also known as: acyl-CoA:16-epivellosimine O-acetyltransferase (cyclizing) Relationships: is a type of acyltransferase activity, transferring groups other than amino-acyl groups [GO:0016747] Sources: EC:2.3.1.160, RHEA:24016 Definition: Catalysis of the reaction: 16-epivellosimine + acetyl-CoA = CoA + vinorine.